{
  "gene": "UniProtKB:P34096",
  "gene_symbol": "RNASE4",
  "gene_name": "Ribonuclease 4",
  "term_label": "extracellular space",
  "term_id": "GO:0005615"
}